{
  "gene_name": "DNA repair-scaffolding protein",
  "gene": "UniProtKB:Q14159",
  "gene_symbol": "SPIDR",
  "term_label": "regulation of establishment of protein localization to chromosome",
  "term_id": "GO:0070202"
}